{
  "gene_name": "Ras-related protein Rab-7b",
  "term_id": "GO:0005770",
  "gene_symbol": "RAB7B",
  "term_label": "late endosome",
  "gene": "UniProtKB:Q96AH8"
}